mutator focus [GO:1990633] (cellular component) Definition: A type of punctate focus localized to the perinuclear region of germline cytoplasm in C. elegans. Mutator foci are required for RNA interference (RNAi) and serve as sites of small inhibitory RNA (siRNA) amplification. As such, proteins that localize to mutator foci include RNA-directed RNA polymerases (RdRPs) and beta-nucleotidyltransferases. Mutator foci are distinct from, but adjacent to or partially overlap, P granules. References: PMID:22713602, PMID:25635455 Sources: GOC:kmv Relationships: is a type of GO:0036464; is part of perinuclear region of cytoplasm [GO:0048471]